{
  "gene_name": "Intraflagellar transport protein 70A",
  "term_id": "GO:0120170",
  "gene_symbol": "IFT70A",
  "gene": "UniProtKB:Q86WT1",
  "term_label": "intraciliary transport particle B binding"
}